{
  "gene": "UniProtKB:Q9NP98",
  "gene_name": "Myozenin-1",
  "gene_symbol": "MYOZ1",
  "term_label": "telethonin binding",
  "term_id": "GO:0031433"
}